{
  "term_id": "GO:0003690",
  "gene_symbol": "CAMTA1",
  "gene": "UniProtKB:Q9Y6Y1",
  "gene_name": "Calmodulin-binding transcription activator 1",
  "term_label": "double-stranded DNA binding"
}